{
  "term_label": "collagen type X trimer",
  "gene_name": "Collagen alpha-1(X) chain",
  "term_id": "GO:0005599",
  "gene_symbol": "COL10A1",
  "gene": "UniProtKB:Q03692"
}